{
  "gene_symbol": "CXCR4",
  "term_label": "calcium-mediated signaling",
  "gene_name": "C-X-C chemokine receptor type 4",
  "term_id": "GO:0019722",
  "gene": "UniProtKB:P61073"
}